{
  "term_label": "unfolded protein binding",
  "gene": "UniProtKB:Q9H009",
  "gene_name": "Nascent polypeptide-associated complex subunit alpha-2",
  "term_id": "GO:0051082",
  "gene_symbol": "NACA2"
}